{
  "term_id": "GO:0031966",
  "gene_symbol": "TMEM70",
  "gene": "UniProtKB:Q9BUB7",
  "gene_name": "Transmembrane protein 70, mitochondrial",
  "term_label": "mitochondrial membrane"
}